{
  "gene_name": "Unconventional myosin-XVIIIb",
  "gene": "UniProtKB:Q8IUG5",
  "term_label": "myosin II complex",
  "gene_symbol": "MYO18B",
  "term_id": "GO:0016460"
}